{
  "gene": "UniProtKB:Q6EBC2",
  "term_id": "GO:0005615",
  "gene_symbol": "IL31",
  "term_label": "extracellular space",
  "gene_name": "Interleukin-31"
}